{
  "term_label": "succinate transmembrane transport",
  "gene_name": "Na(+)_dicarboxylate cotransporter 3",
  "gene": "UniProtKB:Q8WWT9",
  "gene_symbol": "SLC13A3",
  "term_id": "GO:0071422"
}